{
  "gene_name": "Zinc finger protein Gfi-1b",
  "gene": "UniProtKB:Q5VTD9",
  "term_label": "DNA-binding transcription activator activity, RNA polymerase II-specific",
  "term_id": "GO:0001228",
  "gene_symbol": "GFI1B"
}